microtubule-based peroxisome localization [GO:0060152] (biological process) Relationships: is a type of microtubule-based process [GO:0007017]; is a type of GO:0060151 References: PMID:16449325 Sources: GOC:dph Also known as: microtubule-based peroxisome localisation Definition: The microtubule-based process in which a peroxisome is transported to, and/or maintained in, a specific location. A peroxisome is a small membrane-bounded organelle that uses dioxygen (O2) to oxidize organic molecules.